{
  "gene": "UniProtKB:P56915",
  "gene_name": "Homeobox protein goosecoid",
  "term_label": "DNA-binding transcription factor activity, RNA polymerase II-specific",
  "gene_symbol": "GSC",
  "term_id": "GO:0000981"
}